{
  "term_label": "regulation of canonical Wnt signaling pathway",
  "gene_symbol": "RECK",
  "gene_name": "Reversion-inducing cysteine-rich protein with Kazal motifs",
  "term_id": "GO:0060828",
  "gene": "UniProtKB:O95980"
}